3',5'-cyclic-nucleotide phosphodiesterase activity [GO:0004114] (molecular function) Relationships: is a type of cyclic-nucleotide phosphodiesterase activity [GO:0004112] Definition: Catalysis of the reaction: a nucleoside 3',5'-cyclic phosphate + H2O = a nucleoside 5'-phosphate. Also known as: 3',5' cyclic-nucleotide phosphodiesterase activity, cyclic AMP phosphodiesterase activity, 3', 5'-cyclic nucleoside monophosphate phosphodiesterase activity, 3',5'-cyclic-nucleotide 5'-nucleotidohydrolase activity, 3',5'-cyclonucleotide phosphodiesterase activity, 3',5'-nucleotide phosphodiesterase activity, 3': 5'-monophosphate phosphodiesterase (cyclic CMP) activity, 3':5'-cyclic nucleotide 5'-nucleotidohydrolase activity, PDE, cyclic 3',5'-mononucleotide phosphodiesterase activity, cyclic 3',5'-nucleotide phosphodiesterase activity, cyclic 3',5'-phosphodiesterase activity, cyclic 3',5-nucleotide monophosphate phosphodiesterase activity, cyclic nucleotide phosphodiesterase activity, cytidine 3':5'-monophosphate phosphodiesterase (cyclic CMP) activity, nucleoside 3',5'-cyclic phosphate diesterase activity, nucleoside-3',5-monophosphate phosphodiesterase activity References: PMID:35216259 Sources: RHEA:14653 Subtypes: 3',5'-cyclic-AMP phosphodiesterase activity [GO:0004115], 3',5'-cGMP-stimulated cyclic-nucleotide phosphodiesterase activity [GO:0004118], 3',5'-cGMP-inhibited cyclic-nucleotide phosphodiesterase activity [GO:0004119], 3',5'-cyclic-GMP phosphodiesterase activity [GO:0047555]